leaflet of membrane bilayer [GO:0097478] (cellular component) Also known as: membrane leaflet Relationships: is a type of cellular anatomical structure [GO:0110165]; is part of GO:0016020 Definition: Any of the two layers of lipid molecules that constitute a membrane. Sources: GOC:cjm